{
  "gene_name": "G-protein coupled receptor family C group 5 member B",
  "gene": "UniProtKB:Q9NZH0",
  "gene_symbol": "GPRC5B",
  "term_label": "extracellular exosome",
  "term_id": "GO:0070062"
}